{
  "term_id": "GO:0000978",
  "gene_name": "Max-interacting protein 1",
  "term_label": "RNA polymerase II cis-regulatory region sequence-specific DNA binding",
  "gene": "UniProtKB:P50539",
  "gene_symbol": "MXI1"
}